amino-acid betaine metabolic process [GO:0006577] (biological process) Sources: GOC:mah, ISBN:0198506732 Relationships: is a type of modified amino acid metabolic process [GO:0006575] Subtypes: GO:0006578, GO:0006579, carnitine metabolic process [GO:0009437], GO:0052698 Definition: The chemical reactions and pathways involving any betaine, the N-trimethyl derivative of an amino acid. Also known as: betaine metabolic process, betaine metabolism